{
  "term_label": "Unknown cellular component",
  "gene": "UniProtKB:Q8NCL9",
  "term_id": "UNKNOWN:0003",
  "gene_name": "Protein APCDD1-like",
  "gene_symbol": "APCDD1L"
}